{
  "term_id": "GO:0000978",
  "gene": "UniProtKB:Q9H165",
  "gene_symbol": "BCL11A",
  "term_label": "RNA polymerase II cis-regulatory region sequence-specific DNA binding",
  "gene_name": "B-cell lymphoma_leukemia 11A"
}